{
  "gene_name": "PR domain zinc finger protein 8",
  "gene_symbol": "PRDM8",
  "gene": "UniProtKB:Q9NQV8",
  "term_label": "Unknown molecular function",
  "term_id": "UNKNOWN:0001"
}